{
  "gene_symbol": "SIAH1",
  "gene_name": "E3 ubiquitin-protein ligase SIAH1",
  "term_id": "GO:0061630",
  "term_label": "ubiquitin protein ligase activity",
  "gene": "UniProtKB:Q8IUQ4"
}